{
  "gene_symbol": "OR51V1",
  "gene_name": "Olfactory receptor 51V1",
  "gene": "UniProtKB:Q9H2C8",
  "term_id": "GO:0004984",
  "term_label": "olfactory receptor activity"
}